{
  "term_label": "cytoplasm",
  "gene": "UniProtKB:Q6ZVX7",
  "gene_symbol": "NCCRP1",
  "gene_name": "F-box only protein 50",
  "term_id": "GO:0005737"
}